ceramide 1-phosphate transfer activity [GO:1902388] (molecular function) Also known as: ceramide 1-phosphate transporter activity, ceramide 1-phosphate carrier activity, intermembrane ceramide 1-phosphate transfer activity References: PMID:23863933 Sources: GOC:TermGenie Relationships: is a type of phospholipid transfer activity [GO:0120014]; is a type of ceramide transfer activity [GO:0120017]; is part of ceramide 1-phosphate transport [GO:1902389] Definition: Removes a ceramide 1-phosphate from a membrane or a monolayer lipid particle, transports it through the aqueous phase while protected in a hydrophobic pocket, and brings it to an acceptor membrane or lipid particle.